{
  "term_label": "negative regulation of transcription by RNA polymerase II",
  "gene_name": "Zinc finger protein 658",
  "gene_symbol": "ZNF658",
  "term_id": "GO:0000122",
  "gene": "UniProtKB:Q5TYW1"
}